{
  "gene": "UniProtKB:Q9UKJ0",
  "gene_symbol": "PILRB",
  "term_id": "UNKNOWN:0003",
  "term_label": "Unknown cellular component",
  "gene_name": "Paired immunoglobulin-like type 2 receptor beta"
}